positive regulation of myeloid leukocyte differentiation [GO:0002763] (biological process) Definition: Any process that activates or increases the frequency, rate, or extent of myeloid leukocyte differentiation. Sources: GOC:add Also known as: up regulation of myeloid leukocyte differentiation, up-regulation of myeloid leukocyte differentiation, upregulation of myeloid leukocyte differentiation, activation of myeloid leukocyte differentiation, stimulation of myeloid leukocyte differentiation Relationships: is a type of regulation of myeloid leukocyte differentiation [GO:0002761]; is a type of positive regulation of myeloid cell differentiation [GO:0045639]; is a type of GO:1902107; positively regulates myeloid leukocyte differentiation [GO:0002573] Subtypes: GO:0030854, positive regulation of macrophage differentiation [GO:0045651], positive regulation of monocyte differentiation [GO:0045657], positive regulation of osteoclast differentiation [GO:0045672], GO:0060376